{
  "gene": "UniProtKB:P0C7X0",
  "term_label": "Unknown cellular component",
  "gene_symbol": "FAM90A24P",
  "term_id": "UNKNOWN:0003",
  "gene_name": "Putative protein FAM90A24P"
}